{
  "term_label": "heme binding",
  "gene_name": "Hemoglobin subunit gamma-1",
  "gene_symbol": "HBG1",
  "term_id": "GO:0020037",
  "gene": "UniProtKB:P69891"
}